{
  "gene_name": "ADP-ribosylation factor-binding protein GGA2",
  "gene": "UniProtKB:Q9UJY4",
  "term_id": "GO:0005802",
  "term_label": "trans-Golgi network",
  "gene_symbol": "GGA2"
}